{
  "gene": "UniProtKB:Q53GG5",
  "term_label": "filamentous actin",
  "term_id": "GO:0031941",
  "gene_symbol": "PDLIM3",
  "gene_name": "PDZ and LIM domain protein 3"
}